heparin proteoglycan biosynthetic process [GO:0030210] (biological process) Also known as: heparin anabolism, heparin biosynthesis, heparin formation, heparin synthesis, heparan sulfate biosynthetic process References: PMID:22566225 Definition: The chemical reactions and pathways resulting in the formation of heparin proteoglycans, which consist of a core protein linked to a heparin glycosaminoglycan. The heparin chain is composed of the repeating disaccharide unit beta-(1,4)-N-acetyl-D-glucosamine-alpha-(1,4)-hexuronic acid, the former being either sulfated or deacetylated on its amino group as well as sulfated on one of its hydroxyl groups, and the latter being a mixture of sulfated and nonsulfated D-glucuronic and L-iduronic acids. Heparin is similar to heparan sulfate but it contains more N-sulfate and O-sulfate groups. Heparin chains are covalently linked to serine/threonine residues (O-linked) of the core protein via a tetrasaccharide linker sequence (xylose-galactose-galactose-glucuronate). Relationships: is_a heparin proteoglycan metabolic process [GO:0030202]; is a type of protein O-linked glycosylation via xylose [GO:0180064]